{
  "term_label": "JNK cascade",
  "term_id": "GO:0007254",
  "gene_name": "C-Jun-amino-terminal kinase-interacting protein 2",
  "gene": "UniProtKB:Q13387",
  "gene_symbol": "MAPK8IP2"
}